{
  "term_id": "GO:0016020",
  "term_label": "membrane",
  "gene_name": "Neuroendocrine convertase 2",
  "gene_symbol": "PCSK2",
  "gene": "UniProtKB:P16519"
}